{
  "gene": "UniProtKB:Q9Y3Q7",
  "term_label": "proteolysis",
  "gene_symbol": "ADAM18",
  "term_id": "GO:0006508",
  "gene_name": "Disintegrin and metalloproteinase domain-containing protein 18"
}